{
  "term_id": "GO:0030182",
  "gene_symbol": "WNT8A",
  "term_label": "neuron differentiation",
  "gene": "UniProtKB:Q9H1J5",
  "gene_name": "Protein Wnt-8a"
}